{
  "term_id": "GO:0016358",
  "gene_name": "Proto-oncogene DBL",
  "gene": "UniProtKB:P10911",
  "term_label": "dendrite development",
  "gene_symbol": "MCF2"
}